negative regulation of xyloglucan catabolic process [GO:2000952] (biological process) Definition: Any process that stops, prevents or reduces the frequency, rate or extent of xyloglucan catabolic process. Also known as: negative regulation of xyloglucan catabolism Sources: GOC:mengo_curators Relationships: is a type of GO:2000951; is a type of negative regulation of hemicellulose catabolic process [GO:2000989]; negatively regulates xyloglucan catabolic process [GO:2000899]